{
  "term_id": "GO:0071345",
  "term_label": "cellular response to cytokine stimulus",
  "gene_name": "Interferon-induced protein with tetratricopeptide repeats 3",
  "gene_symbol": "IFIT3",
  "gene": "UniProtKB:O14879"
}